{
  "gene_symbol": "KRT72",
  "term_label": "intermediate filament organization",
  "gene": "UniProtKB:Q14CN4",
  "term_id": "GO:0045109",
  "gene_name": "Keratin, type II cytoskeletal 72"
}